{
  "gene_symbol": "FAM98A",
  "term_label": "Unknown biological process",
  "gene": "UniProtKB:Q8NCA5",
  "gene_name": "Protein FAM98A",
  "term_id": "UNKNOWN:0002"
}